{
  "term_label": "negative regulation of translation",
  "gene_symbol": "EIF2AK2",
  "gene_name": "Interferon-induced, double-stranded RNA-activated protein kinase",
  "term_id": "GO:0017148",
  "gene": "UniProtKB:P19525"
}